{
  "term_label": "Unknown biological process",
  "term_id": "UNKNOWN:0002",
  "gene_symbol": "RTBDN",
  "gene_name": "Retbindin",
  "gene": "UniProtKB:Q9BSG5"
}